{
  "gene": "UniProtKB:O60938",
  "term_label": "Unknown biological process",
  "term_id": "UNKNOWN:0002",
  "gene_symbol": "KERA",
  "gene_name": "Keratocan"
}